{
  "gene_name": "Dynein axonemal assembly factor 3",
  "gene_symbol": "DNAAF3",
  "term_id": "GO:0044458",
  "term_label": "motile cilium assembly",
  "gene": "UniProtKB:Q8N9W5"
}